cuticle pigmentation [GO:0048067] (biological process) Regulation: regulated by regulation of cuticle pigmentation [GO:0048079]; negatively regulated by negative regulation of cuticle pigmentation [GO:0048080]; positively regulated by positive regulation of cuticle pigmentation [GO:0048081] Subtypes: adult chitin-containing cuticle pigmentation [GO:0048085] Relationships: is a type of developmental pigmentation [GO:0048066]; is part of cuticle development [GO:0042335] Sources: GOC:jid Definition: Establishment of a pattern of pigment in the cuticle of an organism.